positive regulation of double-strand break repair [GO:2000781] (biological process) Relationships: is a type of positive regulation of DNA repair [GO:0045739]; is a type of GO:2000779; positively regulates double-strand break repair [GO:0006302] Definition: Any process that activates or increases the frequency, rate or extent of double-strand break repair. Sources: GOC:BHF Subtypes: positive regulation of double-strand break repair via homologous recombination [GO:1905168], positive regulation of double-strand break repair via nonhomologous end joining [GO:2001034]